{
  "gene": "UniProtKB:Q13324",
  "gene_symbol": "CRHR2",
  "gene_name": "Corticotropin-releasing factor receptor 2",
  "term_id": "GO:0017046",
  "term_label": "peptide hormone binding"
}